{
  "gene_symbol": "CDH7",
  "gene": "UniProtKB:Q9ULB5",
  "gene_name": "Cadherin-7",
  "term_id": "GO:0007043",
  "term_label": "cell-cell junction assembly"
}